{
  "gene": "UniProtKB:Q96SK2",
  "gene_name": "Transmembrane protein 209",
  "gene_symbol": "TMEM209",
  "term_label": "Unknown molecular function",
  "term_id": "UNKNOWN:0001"
}